{
  "gene": "UniProtKB:Q9HAU8",
  "term_id": "GO:0006508",
  "gene_name": "Aminopeptidase RNPEPL1",
  "gene_symbol": "RNPEPL1",
  "term_label": "proteolysis"
}